{
  "gene": "UniProtKB:Q96BI3",
  "gene_name": "Gamma-secretase subunit APH-1A",
  "gene_symbol": "APH1A",
  "term_id": "GO:0030674",
  "term_label": "protein-macromolecule adaptor activity"
}